{
  "term_id": "GO:0004458",
  "gene_name": "Probable D-lactate dehydrogenase, mitochondrial",
  "gene_symbol": "LDHD",
  "gene": "UniProtKB:Q86WU2",
  "term_label": "D-lactate dehydrogenase (cytochrome) activity"
}